{
  "term_label": "axoneme assembly",
  "term_id": "GO:0035082",
  "gene_name": "Radial spoke head protein 6 homolog A",
  "gene": "UniProtKB:Q9H0K4",
  "gene_symbol": "RSPH6A"
}